{
  "term_label": "positive regulation of cell adhesion",
  "gene": "UniProtKB:Q9Y5U5",
  "gene_name": "Tumor necrosis factor receptor superfamily member 18",
  "term_id": "GO:0045785",
  "gene_symbol": "TNFRSF18"
}